H3 histamine receptor binding [GO:0031809] (molecular function) Definition: Binding to a H3 histamine receptor. Sources: GOC:mah, GOC:nln Relationships: is_a G protein-coupled histamine receptor binding [GO:0031806] Also known as: H3 histamine receptor ligand